{
  "term_id": "GO:0006357",
  "gene_name": "Zinc finger protein 77",
  "term_label": "regulation of transcription by RNA polymerase II",
  "gene_symbol": "ZNF77",
  "gene": "UniProtKB:Q15935"
}